{
  "gene": "UniProtKB:P14616",
  "term_id": "GO:0008286",
  "gene_symbol": "INSRR",
  "term_label": "insulin receptor signaling pathway",
  "gene_name": "Insulin receptor-related protein"
}